{
  "term_id": "GO:0005737",
  "gene_name": "LIM domain kinase 2",
  "gene_symbol": "LIMK2",
  "term_label": "cytoplasm",
  "gene": "UniProtKB:P53671"
}